neurotransmitter-mediated guidance of interneurons involved in substrate-independent cerebral cortex tangential migration [GO:0021845] (BP) References: PMID:12626695 Sources: GOC:cls, GOC:dgh, GOC:dph, GOC:jid, GO_REF:0000021 Relationships: is_a GO:0030334; is part of substrate-independent telencephalic tangential interneuron migration [GO:0021843] Definition: The response of migrating interneurons to neurotransmitters that alter electrical activity in cells in calcium dependent manner.